folic acid receptor activity [GO:0061714] (molecular function) Definition: Combining selectively with extracellular folic acid and delivering it into the cell via endocytosis. Also known as: folate receptor activity Sources: GOC:BHF, GOC:hal Relationships: is a type of GO:0038024; is part of folic acid transport [GO:0015884]; is part of cellular response to folic acid [GO:0071231]; has part folic acid binding [GO:0005542]